{
  "gene_name": "Tripartite motif-containing protein 49D",
  "gene_symbol": "TRIM49D1",
  "gene": "UniProtKB:C9J1S8",
  "term_id": "GO:0045087",
  "term_label": "innate immune response"
}